{
  "gene": "UniProtKB:Q53T59",
  "term_id": "UNKNOWN:0003",
  "term_label": "Unknown cellular component",
  "gene_name": "HCLS1-binding protein 3",
  "gene_symbol": "HS1BP3"
}